{
  "gene_symbol": "ETFDH",
  "term_label": "electron-transferring-flavoprotein dehydrogenase activity",
  "gene": "UniProtKB:Q16134",
  "term_id": "GO:0004174",
  "gene_name": "Electron transfer flavoprotein-ubiquinone oxidoreductase, mitochondrial"
}